{
  "term_label": "double-strand break repair via synthesis-dependent strand annealing",
  "gene_symbol": "RAD54L",
  "gene": "UniProtKB:Q92698",
  "gene_name": "DNA repair and recombination protein RAD54-like",
  "term_id": "GO:0045003"
}